{
  "term_label": "Unknown molecular function",
  "term_id": "UNKNOWN:0001",
  "gene": "UniProtKB:A6NGB7",
  "gene_name": "Transmembrane protein 221",
  "gene_symbol": "TMEM221"
}